chromatin extrusion motor activity [GO:0140584] (molecular function) References: PMID:23074191, PMID:26499245, PMID:27210764 Definition: A DNA translocase activity that folds chromosomal DNA and catalytically extends the newly formed loop, driven by ATP hydrolysis. Relationships: is a type of DNA translocase activity [GO:0015616]; is part of chromatin looping [GO:0140588] Also known as: chromatin extrusion activity